alpha5-beta1 integrin-endostatin complex [GO:0071115] (cellular component) References: PMID:12682293 Also known as: ITGA5-ITGB1-CAL4A3 complex Relationships: is a type of plasma membrane protein complex [GO:0098797] Definition: A protein complex that consists of an alpha5-beta1 integrin complex bound to endostatin, the NC1 domain of the alpha1 chain of type XVIII collagen.